{
  "gene": "UniProtKB:Q6ZMY3",
  "term_label": "nucleus",
  "gene_symbol": "SPOCD1",
  "gene_name": "SPOC domain-containing protein 1",
  "term_id": "GO:0005634"
}